{
  "gene_name": "Splicing factor 45",
  "gene_symbol": "RBM17",
  "gene": "UniProtKB:Q96I25",
  "term_label": "Unknown cellular component",
  "term_id": "UNKNOWN:0003"
}